{
  "term_label": "calcium-dependent protein binding",
  "gene_name": "Protein S100-P",
  "gene_symbol": "S100P",
  "term_id": "GO:0048306",
  "gene": "UniProtKB:P25815"
}